wax-ester hydrolase activity [GO:0050398] (molecular function) Sources: EC:3.1.1.50, MetaCyc:WAX-ESTER-HYDROLASE-RXN Relationships: is a type of carboxylic ester hydrolase activity [GO:0052689] Definition: Catalysis of the reaction: a wax ester + H2O = a long-chain alcohol + a long-chain carboxylate. Also known as: jojoba wax esterase, WEH, wax-ester acylhydrolase activity